nitrobenzene metabolic process [GO:0018916] (biological process) Definition: The chemical reactions and pathways involving nitrobenzene (nitrobenzol), a derivative of benzene with an NO2 group attached to the ring. It is a yellow aromatic liquid used in perfumery and manufactured in large quantities in the preparation of aniline. Also known as: nitrobenzene metabolism Relationships: is a type of benzene-containing compound metabolic process [GO:0042537] Subtypes: GO:1900998, nitrobenzene biosynthetic process [GO:1900999] Sources: GOC:curators